{
  "gene_symbol": "OR13C2",
  "gene_name": "Olfactory receptor 13C2",
  "gene": "UniProtKB:Q8NGS9",
  "term_label": "olfactory receptor activity",
  "term_id": "GO:0004984"
}